{
  "gene_symbol": "SLC27A4",
  "gene_name": "Long-chain fatty acid transport protein 4",
  "term_label": "endoplasmic reticulum membrane",
  "term_id": "GO:0005789",
  "gene": "UniProtKB:Q6P1M0"
}